{
  "term_id": "GO:0000981",
  "gene": "UniProtKB:P78413",
  "gene_symbol": "IRX4",
  "gene_name": "Iroquois-class homeodomain protein IRX-4",
  "term_label": "DNA-binding transcription factor activity, RNA polymerase II-specific"
}